symbiont-mediated suppression of host JAK-STAT cascade via inhibition of STAT2 activity [GO:0039564] (biological process) Relationships: is a type of symbiont-mediated suppression of host JAK-STAT cascade via inhibition of STAT activity [GO:0039562] Definition: A process in which a symbiont interferes with, inhibits or disrupt a JAK-STAT signal cascade in the host organism by reducing the activity of host STAT2 (signal transducer and activator of transcription 2). References: PMID:32699158 Note: This term is for annotation of symbiont proteins that counteract the host innate immune response. Also known as: disruption by virus of host JAK-STAT cascade via inhibition of STAT2 activity, inhibition by virus of host STAT2 activity, inhibition of host STAT2 by virus, suppression by virus of host JAK-STAT cascade via inhibition of STAT2 activity, suppression by virus of host STAT2 activity